{
  "gene": "UniProtKB:Q92917",
  "gene_symbol": "GPKOW",
  "gene_name": "G-patch domain and KOW motifs-containing protein",
  "term_label": "mRNA splicing, via spliceosome",
  "term_id": "GO:0000398"
}